polyadic synapse [GO:0098979] (cellular component) Definition: A synapse consisting of a single presynapse and multiple postsynapses. These postsynapses may come from the same cell of from different cells. Polyadic synapses are common in arthropod and nematode central nervous systems. Relationships: is a type of synapse [GO:0045202] References: PMID:26780543